{
  "term_label": "cytoplasm",
  "gene_name": "Geranylgeranyl transferase type-2 subunit alpha",
  "term_id": "GO:0005737",
  "gene_symbol": "RABGGTA",
  "gene": "UniProtKB:Q92696"
}